positive regulation of exit from mitosis [GO:0031536] (biological process) Sources: GOC:mah Definition: Any process that activates or increases the rate of progression from anaphase/telophase (high mitotic CDK activity) to G1 (low mitotic CDK activity). Also known as: up regulation of exit from mitosis, up-regulation of exit from mitosis, upregulation of exit from mitosis, activation of exit from mitosis, stimulation of exit from mitosis Relationships: is a type of regulation of exit from mitosis [GO:0007096]; is a type of positive regulation of mitotic cell cycle phase transition [GO:1901992]; RO_0002213 exit from mitosis [GO:0010458]